peptidoglycan L,D-transpeptidase activity [GO:0071972] (molecular function) Definition: Catalysis of the reaction: 2 a peptidoglycan dimer (tetrapeptide) + 3 H2O = a peptidoglycan tetramer with L,D cross-links (L-Lys-D-Asn-L-Lys) + di-trans,poly-cis-undecaprenyl diphosphate + 4 D-alanine. Sources: MetaCyc:RXN-11349 Relationships: is_a serine-type carboxypeptidase activity [GO:0004185]